regulation of establishment of T cell polarity [GO:1903903] (BP) Subtypes: negative regulation of establishment of T cell polarity [GO:1903904], positive regulation of establishment of T cell polarity [GO:1903905] Relationships: is a type of GO:2000114; regulates GO:0001768 References: PMID:23575248 Sources: GOC:TermGenie, GOC:als, GO_REF:0000058 Also known as: regulation of T cell polarization, regulation of T lymphocyte polarization, regulation of T-cell polarization, regulation of establishment of T lymphocyte polarity, regulation of establishment of T-cell polarity, regulation of establishment of T-lymphocyte polarity Definition: Any process that modulates the frequency, rate or extent of establishment of T cell polarity.